{
  "term_id": "UNKNOWN:0003",
  "term_label": "Unknown cellular component",
  "gene_name": "Endonuclease domain-containing 1 protein",
  "gene": "UniProtKB:O94919",
  "gene_symbol": "ENDOD1"
}